{
  "gene_symbol": "DPH3",
  "gene": "UniProtKB:Q96FX2",
  "term_id": "GO:0005829",
  "term_label": "cytosol",
  "gene_name": "Diphthamide biosynthesis protein 3"
}